{
  "term_label": "histone H3K4me/H3K4me2/H3K4me3 demethylase activity",
  "gene_symbol": "KDM5D",
  "gene": "UniProtKB:Q9BY66",
  "term_id": "GO:0034647",
  "gene_name": "Lysine-specific demethylase 5D"
}